{
  "term_label": "DNA helicase activity",
  "term_id": "GO:0003678",
  "gene_symbol": "RUVBL2",
  "gene_name": "RuvB-like 2",
  "gene": "UniProtKB:Q9Y230"
}